{
  "gene_symbol": "IGHD3-3",
  "gene": "UniProtKB:A0A0J9YWD0",
  "term_label": "Unknown cellular component",
  "gene_name": "Immunoglobulin heavy diversity 3-3 (Fragment)",
  "term_id": "UNKNOWN:0003"
}